negative regulation of chaperone-mediated autophagy [GO:1904715] (biological process) Definition: Any process that stops, prevents or reduces the frequency, rate or extent of chaperone-mediated autophagy. References: PMID:20176123 Sources: GOC:PARL, GOC:TermGenie, GOC:pad, GO_REF:0000058 Also known as: down regulation of chaperone-mediated autophagy, down-regulation of chaperone-mediated autophagy, downregulation of chaperone-mediated autophagy, inhibition of chaperone-mediated autophagy, down regulation of CMA, down-regulation of CMA, downregulation of CMA, inhibition of CMA, negative regulation of CMA Relationships: is a type of negative regulation of autophagy [GO:0010507]; is a type of GO:0042177; is_a regulation of chaperone-mediated autophagy [GO:1904714]; RO_0002212 chaperone-mediated autophagy [GO:0061684]